{
  "gene_name": "Protein KRI1 homolog",
  "term_id": "GO:0000447",
  "term_label": "endonucleolytic cleavage in ITS1 to separate SSU-rRNA from 5.8S rRNA and LSU-rRNA from tricistronic rRNA transcript (SSU-rRNA, 5.8S rRNA, LSU-rRNA)",
  "gene": "UniProtKB:Q8N9T8",
  "gene_symbol": "KRI1"
}